{
  "term_id": "GO:0045087",
  "term_label": "innate immune response",
  "gene": "UniProtKB:Q6ZMU5",
  "gene_symbol": "TRIM72",
  "gene_name": "Tripartite motif-containing protein 72"
}